{
  "gene_name": "Ferric-chelate reductase 1",
  "gene": "UniProtKB:Q6ZNA5",
  "gene_symbol": "FRRS1",
  "term_id": "GO:0016020",
  "term_label": "membrane"
}